{
  "gene": "UniProtKB:P28223",
  "gene_symbol": "HTR2A",
  "term_label": "plasma membrane",
  "gene_name": "5-hydroxytryptamine receptor 2A",
  "term_id": "GO:0005886"
}